{
  "gene": "UniProtKB:P62952",
  "term_id": "UNKNOWN:0003",
  "gene_symbol": "BLCAP",
  "gene_name": "Bladder cancer-associated protein",
  "term_label": "Unknown cellular component"
}